magnesium chelatase activity [GO:0016851] (molecular function) Definition: Catalysis of the reaction: ATP + H2O + Mg2+ + protoporphyrin IX = ADP + 3 H+ + Mg-protoporphyrin IX + phosphate. Sources: RHEA:13961 Relationships: is a type of ligase activity, forming nitrogen-metal bonds, forming coordination complexes [GO:0051003] Also known as: Mg-chelatase activity, Mg-protoporphyrin IX chelatase activity, Mg-protoporphyrin IX magnesio-lyase activity, Mg-protoporphyrin IX magnesium-lyase activity, magnesium-chelatase activity, magnesium-protoporphyrin IX chelatase activity, magnesium-protoporphyrin chelatase activity, protoporphyrin IX Mg-chelatase activity, protoporphyrin IX magnesium-chelatase activity